methylation [GO:0032259] (biological process) Subtypes: macromolecule methylation [GO:0043414] Sources: GOC:mah Definition: The process in which a methyl group is covalently attached to a molecule. Relationships: is a type of metabolic process [GO:0008152]